positive regulation of transcription initiation by RNA polymerase II [GO:0060261] (biological process) Sources: GOC:dph, GOC:tb, GOC:txnOH Subtypes: positive regulation of RNA polymerase II transcription preinitiation complex assembly [GO:0045899] Also known as: positive regulation of transcription initiation from RNA polymerase II promoter Relationships: is a type of positive regulation of transcription by RNA polymerase II [GO:0045944]; is a type of GO:0060260; is a type of GO:2000144; positively regulates GO:0006367 Definition: Any process that increases the rate, frequency or extent of a process involved in starting transcription from an RNA polymerase II promoter.